negative regulation of lymphocyte differentiation [GO:0045620] (biological process) Note: Note that immunologists typically use the word 'development' to refer to cells of B or T cell lineages undergoing the process that GO describes as 'cell differentiation'. Definition: Any process that stops, prevents, or reduces the frequency, rate or extent of lymphocyte differentiation. Subtypes: GO:0032824, negative regulation of B cell differentiation [GO:0045578], negative regulation of T cell differentiation [GO:0045581] Relationships: is a type of regulation of lymphocyte differentiation [GO:0045619]; is a type of GO:0051250; is a type of negative regulation of leukocyte differentiation [GO:1902106]; negatively regulates lymphocyte differentiation [GO:0030098] Also known as: down regulation of lymphocyte differentiation, down-regulation of lymphocyte differentiation, downregulation of lymphocyte differentiation, inhibition of lymphocyte differentiation, negative regulation of lymphocyte development Sources: GOC:go_curators